{
  "term_id": "UNKNOWN:0002",
  "gene": "UniProtKB:Q13268",
  "gene_symbol": "DHRS2",
  "gene_name": "Dehydrogenase_reductase SDR family member 2, mitochondrial",
  "term_label": "Unknown biological process"
}